{
  "gene_name": "Centrosomal protein of 44 kDa",
  "term_id": "GO:0000922",
  "gene": "UniProtKB:Q9C0F1",
  "term_label": "spindle pole",
  "gene_symbol": "CEP44"
}